{
  "term_label": "mitochondrial inner membrane",
  "gene": "UniProtKB:Q96E52",
  "gene_name": "Metalloendopeptidase OMA1, mitochondrial",
  "gene_symbol": "OMA1",
  "term_id": "GO:0005743"
}